{
  "gene_symbol": "ELP2",
  "gene": "UniProtKB:Q6IA86",
  "term_label": "Unknown molecular function",
  "term_id": "UNKNOWN:0001",
  "gene_name": "Elongator complex protein 2"
}